{
  "gene_symbol": "IHH",
  "gene_name": "Indian hedgehog protein",
  "gene": "UniProtKB:Q14623",
  "term_id": "GO:0007224",
  "term_label": "smoothened signaling pathway"
}